{
  "term_id": "GO:0007411",
  "gene": "UniProtKB:P54762",
  "gene_name": "Ephrin type-B receptor 1",
  "gene_symbol": "EPHB1",
  "term_label": "axon guidance"
}